spermine catabolic process [GO:0046208] (BP) References: PMID:12141946 Also known as: spermine breakdown, spermine catabolism, spermine degradation Relationships: is a type of polyamine catabolic process [GO:0006598]; is a type of spermine metabolic process [GO:0008215] Definition: The chemical reactions and pathways resulting in the breakdown of spermine, a polybasic amine found in human sperm, in ribosomes and in some viruses and involved in nucleic acid packaging.